rRNA catabolic process [GO:0016075] (biological process) Sources: GOC:ai Definition: The chemical reactions and pathways resulting in the breakdown of rRNA, ribosomal RNA, a structural constituent of ribosomes. Subtypes: cytoplasmic polyadenylation-dependent rRNA catabolic process [GO:0035760], GO:0070651 Regulation: regulated by regulation of rRNA catabolic process [GO:1902374] Also known as: rRNA breakdown, rRNA catabolism, rRNA degradation Relationships: is a type of RNA catabolic process [GO:0006401]; is a type of rRNA metabolic process [GO:0016072]